{
  "gene_name": "b(0,+)-type amino acid transporter 1",
  "term_label": "amino acid transmembrane transport",
  "gene": "UniProtKB:P82251",
  "term_id": "GO:0003333",
  "gene_symbol": "SLC7A9"
}